{
  "gene": "UniProtKB:Q99735",
  "term_label": "leukotriene biosynthetic process",
  "term_id": "GO:0019370",
  "gene_name": "Microsomal glutathione S-transferase 2",
  "gene_symbol": "MGST2"
}